detection of increased carbon dioxide by chemoreceptor signaling [GO:0003021] (biological process) Also known as: detection of increased carbon dioxide by chemoreceptor signalling Definition: The process in which information about the levels of carbon dioxide are received and are converted to a molecular signal by chemoreceptors in the carotid bodies and the aortic bodies. Sources: GOC:mtg_cardio, ISBN:0323031951 Subtypes: GO:0003034, detection of increased carbon dioxide by carotid body chemoreceptor signaling [GO:0003035] Relationships: is a type of detection of carbon dioxide [GO:0003031]; is part of GO:0002007